{
  "term_id": "GO:0005615",
  "term_label": "extracellular space",
  "gene_name": "C-C motif chemokine 18",
  "gene": "UniProtKB:P55774",
  "gene_symbol": "CCL18"
}